{
  "term_label": "negative regulation of DNA-templated transcription",
  "gene": "UniProtKB:Q9P1T7",
  "gene_name": "MyoD family inhibitor domain-containing protein",
  "term_id": "GO:0045892",
  "gene_symbol": "MDFIC"
}